positive regulation of NK T cell proliferation [GO:0051142] (biological process) Definition: Any process that activates or increases the frequency, rate or extent of natural killer T cell proliferation. Also known as: positive regulation of NK T lymphocyte proliferation, positive regulation of NK T-cell proliferation, positive regulation of NK T-lymphocyte proliferation, positive regulation of NKT cell proliferation, positive regulation of NT cell proliferation, positive regulation of natural T cell proliferation, positive regulation of natural killer T cell proliferation, up regulation of NK T cell proliferation, up-regulation of NK T cell proliferation, upregulation of NK T cell proliferation, activation of NK T cell proliferation, stimulation of NK T cell proliferation Relationships: is a type of positive regulation of alpha-beta T cell proliferation [GO:0046641]; is a type of positive regulation of NK T cell activation [GO:0051135]; is a type of regulation of NK T cell proliferation [GO:0051140]; positively regulates GO:0001866 References: PMID:12154375, PMID:9133426 Sources: ISBN:0781735149